glucose catabolic process to pyruvate [GO:0061718] (biological process) Definition: The chemical reactions and pathways resulting in the breakdown of glucose, with the production of pyruvate. Sources: GOC:dph Also known as: glucose catabolism to pyruvate Relationships: is a type of GO:0006007; is a type of pyruvate metabolic process [GO:0006090] Subtypes: canonical glycolysis [GO:0061621], GO:0061633, Entner-Doudoroff pathway through gluconate to D-glyceraldehyde [GO:0061680], glucose catabolic process to pyruvate utilizing ADP [GO:0061719]